{
  "gene": "UniProtKB:Q4G0X9",
  "term_label": "heart looping",
  "term_id": "GO:0001947",
  "gene_name": "Coiled-coil domain-containing protein 40",
  "gene_symbol": "CCDC40"
}